{
  "term_label": "membrane",
  "gene": "UniProtKB:Q92817",
  "gene_symbol": "EVPL",
  "term_id": "GO:0016020",
  "gene_name": "Envoplakin"
}